{
  "gene_name": "Melanoma-associated antigen B5",
  "term_id": "GO:0005634",
  "gene": "UniProtKB:Q9BZ81",
  "term_label": "nucleus",
  "gene_symbol": "MAGEB5"
}